negative regulation of plasmatocyte differentiation [GO:0045614] (biological process) Definition: Any process that stops, prevents, or reduces the frequency, rate or extent of plasmatocyte differentiation. Sources: GOC:go_curators Relationships: is a type of negative regulation of hemocyte differentiation [GO:0045611]; is a type of regulation of plasmatocyte differentiation [GO:0045613]; negatively regulates plasmatocyte differentiation [GO:0042387] Also known as: down regulation of plasmatocyte differentiation, down-regulation of plasmatocyte differentiation, downregulation of plasmatocyte differentiation, inhibition of plasmatocyte differentiation